{
  "term_id": "UNKNOWN:0003",
  "gene_name": "Olfactory receptor 4F6",
  "gene_symbol": "OR4F6",
  "gene": "UniProtKB:Q8NGB9",
  "term_label": "Unknown cellular component"
}